{
  "gene_symbol": "RASSF6",
  "gene": "UniProtKB:Q6ZTQ3",
  "term_label": "signal transduction",
  "term_id": "GO:0007165",
  "gene_name": "Ras association domain-containing protein 6"
}